negative regulation of intestinal lipid absorption [GO:1904730] (biological process) References: PMID:18768481 Sources: GOC:TermGenie, GO_REF:0000058 Relationships: is a type of GO:1904479; is a type of regulation of intestinal lipid absorption [GO:1904729]; negatively regulates GO:0098856 Subtypes: negative regulation of intestinal phytosterol absorption [GO:0010949], negative regulation of intestinal cholesterol absorption [GO:0045796] Definition: Any process that stops, prevents or reduces the frequency, rate or extent of intestinal lipid absorption. Also known as: down regulation of intestinal lipid absorption, down-regulation of intestinal lipid absorption, downregulation of intestinal lipid absorption, inhibition of intestinal lipid absorption